{
  "term_id": "GO:0030335",
  "gene_name": "C-C motif chemokine 1",
  "term_label": "positive regulation of cell migration",
  "gene_symbol": "CCL1",
  "gene": "UniProtKB:P22362"
}